{
  "term_label": "proteolysis",
  "term_id": "GO:0006508",
  "gene_symbol": "NRIP3",
  "gene_name": "Nuclear receptor-interacting protein 3",
  "gene": "UniProtKB:Q9NQ35"
}